{
  "gene_name": "Serum amyloid A-1 protein",
  "gene": "UniProtKB:P0DJI8",
  "term_id": "GO:0048246",
  "term_label": "macrophage chemotaxis",
  "gene_symbol": "SAA1"
}